{
  "term_id": "GO:0005886",
  "gene_symbol": "GPR135",
  "gene_name": "G-protein coupled receptor 135",
  "term_label": "plasma membrane",
  "gene": "UniProtKB:Q8IZ08"
}